beta-alanine transmembrane transporter activity [GO:0001761] (MF) Relationships: is a type of GO:0015175; is a type of carboxylic acid transmembrane transporter activity [GO:0046943]; is part of beta-alanine transport [GO:0001762] Sources: GOC:hjd Definition: Enables the transfer of beta-alanine from one side of a membrane to the other. Beta-alanine is 3-aminopropanoic acid. Also known as: beta-alanine transporter activity